{
  "term_id": "GO:0005783",
  "term_label": "endoplasmic reticulum",
  "gene_name": "Piezo-type mechanosensitive ion channel component 1",
  "gene_symbol": "PIEZO1",
  "gene": "UniProtKB:Q92508"
}